{
  "term_id": "GO:0005634",
  "gene": "UniProtKB:Q92949",
  "gene_name": "Forkhead box protein J1",
  "gene_symbol": "FOXJ1",
  "term_label": "nucleus"
}